{
  "gene": "UniProtKB:Q92664",
  "term_id": "GO:0005634",
  "gene_symbol": "GTF3A",
  "term_label": "nucleus",
  "gene_name": "Transcription factor IIIA"
}